{
  "term_label": "cytoplasm",
  "gene_name": "Glucosamine-6-phosphate isomerase 1",
  "gene_symbol": "GNPDA1",
  "term_id": "GO:0005737",
  "gene": "UniProtKB:P46926"
}